{
  "term_id": "GO:0031145",
  "gene": "UniProtKB:Q9UJX5",
  "gene_symbol": "ANAPC4",
  "gene_name": "Anaphase-promoting complex subunit 4",
  "term_label": "anaphase-promoting complex-dependent catabolic process"
}